{
  "gene_symbol": "HSD11B1",
  "term_id": "GO:0006706",
  "term_label": "steroid catabolic process",
  "gene": "UniProtKB:P28845",
  "gene_name": "11-beta-hydroxysteroid dehydrogenase 1"
}